{
  "term_id": "GO:0015269",
  "term_label": "calcium-activated potassium channel activity",
  "gene": "UniProtKB:Q9P0L9",
  "gene_name": "Polycystin-2-like protein 1",
  "gene_symbol": "PKD2L1"
}